{
  "term_label": "fatty acid beta-oxidation",
  "gene_symbol": "ABCD2",
  "gene_name": "ATP-binding cassette sub-family D member 2",
  "term_id": "GO:0006635",
  "gene": "UniProtKB:Q9UBJ2"
}